purine-containing compound metabolic process [GO:0072521] (biological process) Also known as: purine and derivative metabolic process, purine-containing compound metabolism Subtypes: GO:0006144, GO:0006163, acyl-CoA metabolic process [GO:0006637], coenzyme A metabolic process [GO:0015936], purine nucleoside bisphosphate metabolic process [GO:0034032], GO:0042278, GO:0046415, purine alkaloid metabolic process [GO:0046446], purine-containing compound biosynthetic process [GO:0072522], purine-containing compound catabolic process [GO:0072523] Sources: GOC:mah Definition: The chemical reactions and pathways involving a purine-containing compound, i.e. any compound that contains purine or a formal derivative thereof. Relationships: is_a metabolic process [GO:0008152]